{
  "gene": "UniProtKB:P52799",
  "gene_name": "Ephrin-B2",
  "term_label": "blood vessel morphogenesis",
  "gene_symbol": "EFNB2",
  "term_id": "GO:0048514"
}